{
  "term_label": "adenylate cyclase-inhibiting G protein-coupled receptor signaling pathway",
  "gene_name": "Insulin-like 3",
  "gene": "UniProtKB:P51460",
  "gene_symbol": "INSL3",
  "term_id": "GO:0007193"
}